{
  "term_id": "UNKNOWN:0001",
  "gene": "UniProtKB:Q92575",
  "gene_symbol": "UBXN4",
  "term_label": "Unknown molecular function",
  "gene_name": "UBX domain-containing protein 4"
}